aspyridone A biosynthetic process [GO:1901518] (biological process) Definition: The chemical reactions and pathways resulting in the formation of aspyridone A. Sources: GOC:TermGenie, GOC:di Relationships: is a type of polyketide biosynthetic process [GO:0030639]; is a type of GO:0072525 Also known as: aspyridone A anabolism, aspyridone A biosynthesis, aspyridone A formation, aspyridone A synthesis